{
  "term_label": "nucleus",
  "term_id": "GO:0005634",
  "gene_symbol": "MAK",
  "gene_name": "Serine_threonine-protein kinase MAK",
  "gene": "UniProtKB:P20794"
}